{
  "gene_symbol": "RAB8B",
  "term_id": "GO:0030140",
  "term_label": "trans-Golgi network transport vesicle",
  "gene": "UniProtKB:Q92930",
  "gene_name": "Ras-related protein Rab-8B"
}